{
  "gene_symbol": "MGST1",
  "gene": "UniProtKB:P10620",
  "gene_name": "Microsomal glutathione S-transferase 1",
  "term_id": "GO:0005739",
  "term_label": "mitochondrion"
}